{
  "gene_symbol": "STX3",
  "term_id": "GO:0012505",
  "term_label": "endomembrane system",
  "gene_name": "Syntaxin-3",
  "gene": "UniProtKB:Q13277"
}